regulation of smooth muscle cell apoptotic process [GO:0034391] (biological process) Subtypes: GO:0034392, positive regulation of smooth muscle cell apoptotic process [GO:0034393], GO:1905459 Sources: GOC:BHF, GOC:mtg_apoptosis, GOC:rl Definition: Any process that modulates the frequency, rate, or extent of smooth muscle cell apoptotic process. Also known as: regulation of SMC apoptosis, regulation of smooth muscle cell apoptosis Relationships: is a type of GO:0010660; RO_0002211 smooth muscle cell apoptotic process [GO:0034390]